{
  "term_id": "GO:0005829",
  "gene_name": "Cytosolic Fe-S cluster assembly factor NUBP2",
  "gene_symbol": "NUBP2",
  "gene": "UniProtKB:Q9Y5Y2",
  "term_label": "cytosol"
}